{
  "term_id": "GO:0090619",
  "term_label": "meiotic spindle pole",
  "gene_name": "Protein KASH5",
  "gene": "UniProtKB:Q8N6L0",
  "gene_symbol": "KASH5"
}